response to chemical [GO:0042221] (biological process) Definition: Any process that results in a change in state or activity of a cell or an organism (in terms of movement, secretion, enzyme production, gene expression, etc.) as a result of a chemical stimulus. Sources: GOC:jl Also known as: response to chemical stimulus, response to chemical substance Note: Note that this term is in the subset of terms that should not be used for direct gene product annotation. Instead, select a child term or, if no appropriate child term exists, please request a new term. Direct annotations to this term may be amended during annotation QC. Relationships: is a type of response to stimulus [GO:0050896] Subtypes: GO:0001101, response to nutrient [GO:0007584], response to xenobiotic stimulus [GO:0009410], response to toxic substance [GO:0009636], response to hormone [GO:0009725], response to boron-containing substance [GO:0010036], response to metal ion [GO:0010038], GO:0010269, response to cyclopentenone [GO:0010583], response to cycloalkane [GO:0014071], response to pheromone [GO:0019236], response to food [GO:0032094], response to lipid [GO:0033993], response to nicotine [GO:0035094], response to stilbenoid [GO:0035634], response to diuretic [GO:0036270], GO:0036271, GO:0036275, response to antidepressant [GO:0036276], response to anticonvulsant [GO:0036277], response to antibiotic [GO:0046677], response to organophosphorus [GO:0046683], response to arsenic-containing substance [GO:0046685], response to methylmercury [GO:0051597], response to anticoagulant [GO:0061476], GO:0061477, response to platelet aggregation inhibitor [GO:0061478], response to asparaginase [GO:0061480], response to TNF agonist [GO:0061481], response to irinotecan [GO:0061482], cellular response to chemical stimulus [GO:0070887], GO:0071871, response to anesthetic [GO:0072347], response to bismuth [GO:0072700], response to cisplatin [GO:0072718], GO:0072728, GO:0072739, response to topoisomerase inhibitor [GO:0072758], response to phenylpropanoid [GO:0080184], response to antineoplastic agent [GO:0097327], response to carboplatin [GO:0097328], response to antimetabolite [GO:0097329], response to antipsychotic drug [GO:0097332], response to bronchodilator [GO:0097366], response to benzene [GO:1901423], response to toluene [GO:1901424], response to decalin [GO:1901493], response to tetralin [GO:1901498], GO:1901501, response to paraquat [GO:1901562], response to peptide [GO:1901652], response to nitrogen compound [GO:1901698], response to oxygen-containing compound [GO:1901700], response to salt [GO:1902074], response to N-phenylthiourea [GO:1902610], GO:1902617, GO:1902778, GO:1903165, response to cyanide [GO:1903927], response to Aroclor 1254 [GO:1904010], response to Thyroglobulin triiodothyronine [GO:1904016], response to nonylphenol [GO:1904147], response to 3,3',4,4',5-pentachlorobiphenyl [GO:1904610], GO:1904612, GO:1904614, response to dimethyl sulfoxide [GO:1904619], response to tetrachloromethane [GO:1904772], GO:1904880, GO:1990267, GO:1990834